GABA receptor activity [GO:0016917] (molecular function) Note: See also the molecular function term 'neurotransmitter receptor activity ; GO:0030594'. Also known as: 4-aminobutanoate receptor activity, 4-aminobutyrate receptor activity, GABA binding, gamma-aminobutyrate binding, gamma-aminobutyric acid binding, gamma-aminobutyric acid receptor activity Subtypes: GO:0004890, G protein-coupled GABA receptor activity [GO:0004965] References: PMID:10637650 Sources: GOC:jl, GOC:signaling Definition: Combining with gamma-aminobutyric acid (GABA), and transmitting the signal from one side of the membrane to the other to initiate a change in cell activity. (GABA, 4-aminobutyrate) is an amino acid which acts as a neurotransmitter in some organisms. Relationships: is_a GO:0004888